{
  "term_id": "GO:0007010",
  "term_label": "cytoskeleton organization",
  "gene_symbol": "RANBP9",
  "gene": "UniProtKB:Q96S59",
  "gene_name": "Ran-binding protein 9"
}